{
  "term_id": "GO:0007186",
  "gene_symbol": "OR5M10",
  "gene": "UniProtKB:Q6IEU7",
  "gene_name": "Olfactory receptor 5M10",
  "term_label": "G protein-coupled receptor signaling pathway"
}